{
  "gene_symbol": "SLC25A17",
  "gene": "UniProtKB:O43808",
  "term_label": "peroxisomal membrane",
  "gene_name": "Peroxisomal membrane protein PMP34",
  "term_id": "GO:0005778"
}